adenylate cyclase-inhibiting serotonin receptor signaling pathway [GO:0007198] (biological process) Relationships: is a type of adenylate cyclase-inhibiting G protein-coupled receptor signaling pathway [GO:0007193]; is_a GO:0098664; BFO_0000051 Gi/o-coupled serotonin receptor activity [GO:0001586] Also known as: serotonin receptor, adenylate cyclase inhibiting pathway, inhibition of adenylate cyclase activity by serotonin receptor signaling pathway, inhibition of adenylate cyclase activity by serotonin receptor signalling pathway, serotonin receptor, adenylyl cyclase inhibiting pathway Definition: An adenylate cyclase-inhibiting G protein-coupled receptor signaling pathway initiated by serotonin binding to its receptor, and ending with the regulation of a downstream cellular process. Sources: GOC:dph, GOC:mah, GOC:signaling, GOC:tb